regulation of autophagosome assembly [GO:2000785] (biological process) Relationships: is a type of regulation of vacuole organization [GO:0044088]; is a type of GO:1902115; regulates GO:0000045 Definition: Any process that modulates the frequency, rate or extent of autophagosome assembly. Sources: GOC:BHF, GOC:autophagy Subtypes: negative regulation of autophagosome assembly [GO:1902902], positive regulation of autophagosome assembly [GO:2000786] Also known as: regulation of autophagic vacuole assembly, regulation of autophagosome biosynthesis, regulation of autophagosome formation, regulation of PAS formation, regulation of autophagic vacuole formation